{
  "gene_name": "Uncharacterized protein FLJ76381",
  "gene": "UniProtKB:Q8NFD4",
  "term_id": "UNKNOWN:0003",
  "gene_symbol": "Q8NFD4",
  "term_label": "Unknown cellular component"
}